glucuronoxylan biosynthetic process [GO:0010417] (biological process) Definition: The chemical reactions and pathways resulting in the formation of glucuronoxylan, a polymer containing a beta-1,4-linked D-xylose backbone substituted with glucuronic acid residues. Sources: GOC:tair_curators Relationships: is a type of glucuronoxylan metabolic process [GO:0010413]; is a type of xylan biosynthetic process [GO:0045492] Also known as: glucuronoxylan anabolism, glucuronoxylan biosynthesis, glucuronoxylan formation, glucuronoxylan synthesis